hydrogen peroxide metabolic process [GO:0042743] (biological process) Definition: The chemical reactions and pathways involving hydrogen peroxide (H2O2), a potentially harmful byproduct of aerobic cellular respiration which can cause damage to DNA. References: PMID:21734470 Sources: GOC:jl Also known as: H2O2 metabolic process, hydrogen peroxide metabolism Relationships: is a type of GO:0072593 Subtypes: GO:0042744, hydrogen peroxide biosynthetic process [GO:0050665], detoxification of hydrogen peroxide [GO:0061691] Regulation: regulated by GO:0010310; negatively regulated by negative regulation of hydrogen peroxide metabolic process [GO:0010727]